{
  "term_id": "GO:0016230",
  "gene_symbol": "NSMAF",
  "gene": "UniProtKB:Q92636",
  "gene_name": "Protein FAN",
  "term_label": "sphingomyelin phosphodiesterase activator activity"
}